{
  "gene": "UniProtKB:P23921",
  "gene_name": "Ribonucleoside-diphosphate reductase large subunit",
  "term_id": "GO:0005971",
  "term_label": "ribonucleoside-diphosphate reductase complex",
  "gene_symbol": "RRM1"
}